bicyclogermacrene biosynthetic process [GO:1901934] (biological process) Also known as: bicyclogermacrene anabolism, bicyclogermacrene biosynthesis, bicyclogermacrene formation, bicyclogermacrene synthesis Definition: The chemical reactions and pathways resulting in the formation of bicyclogermacrene. References: PMID:22867794 Sources: GOC:TermGenie Relationships: is a type of sesquiterpene biosynthetic process [GO:0051762]